{
  "term_label": "plasma membrane",
  "gene": "UniProtKB:P0DMV9",
  "gene_symbol": "HSPA1B",
  "gene_name": "Heat shock 70 kDa protein 1B",
  "term_id": "GO:0005886"
}